{
  "gene": "UniProtKB:Q9HAW8",
  "term_id": "GO:0019899",
  "gene_name": "UDP-glucuronosyltransferase 1A10",
  "gene_symbol": "UGT1A10",
  "term_label": "enzyme binding"
}